H4 histone acetyltransferase complex [GO:1902562] (cellular component) Definition: A protein complex which is capable of H4 histone acetyltransferase activity. References: PMID:23775086 Sources: GOC:TermGenie, GOC:bhm Also known as: Hpa3 (homo-)dimer, Hpa3 complex Note: An example of this is Hpa2 in yeast [Q06592] in PMID:23775086 [IDA]. Relationships: is a type of histone acetyltransferase complex [GO:0000123] Subtypes: GO:0043189, NSL complex [GO:0044545], MSL complex [GO:0072487], GO:1990331